{
  "gene_symbol": "HSP90B1",
  "term_id": "GO:0036503",
  "gene": "UniProtKB:P14625",
  "gene_name": "Endoplasmin",
  "term_label": "ERAD pathway"
}